{
  "gene_name": "Zinc finger protein 726",
  "term_id": "GO:0000978",
  "gene_symbol": "ZNF726",
  "gene": "UniProtKB:A6NNF4",
  "term_label": "RNA polymerase II cis-regulatory region sequence-specific DNA binding"
}